positive regulation of late endosome to lysosome transport [GO:1902824] (biological process) Also known as: up regulation of late endosome to lysosome transport, up-regulation of late endosome to lysosome transport, upregulation of late endosome to lysosome transport, activation of late endosome to lysosome transport Relationships: is a type of regulation of late endosome to lysosome transport [GO:1902822]; is a type of positive regulation of vacuolar transport [GO:1903337]; positively regulates GO:1902774 References: PMID:23949442 Sources: GOC:PARL, GOC:TermGenie, GOC:pad, GO_REF:0000058 Definition: Any process that activates or increases the frequency, rate or extent of late endosome to lysosome transport.